{
  "term_id": "UNKNOWN:0003",
  "gene_symbol": "TEX47",
  "term_label": "Unknown cellular component",
  "gene_name": "Testis-expressed protein 47",
  "gene": "UniProtKB:Q8TBZ9"
}